{
  "gene_symbol": "SEC24C",
  "gene_name": "Protein transport protein Sec24C",
  "term_id": "GO:0070971",
  "term_label": "endoplasmic reticulum exit site",
  "gene": "UniProtKB:P53992"
}